peptidyl-lysine N6-palmitoyltransferase activity [GO:0018031] (molecular function) Definition: Catalysis of the transfer of a palmitoyl group to the N6 nitrogen atom on a lysine residue of a peptide or protein molecule. References: PMID:29074776 Sources: GOC:mah Subtypes: GO:0140771, GO:0140772 Relationships: is a type of N-acyltransferase activity [GO:0016410]; is a type of catalytic activity, acting on a protein [GO:0140096]